{
  "gene": "UniProtKB:Q9HBE1",
  "gene_name": "POZ-, AT hook-, and zinc finger-containing protein 1",
  "term_id": "GO:0002682",
  "gene_symbol": "PATZ1",
  "term_label": "regulation of immune system process"
}